{
  "gene_name": "Nucleoside diphosphate kinase 7",
  "term_id": "GO:0005813",
  "term_label": "centrosome",
  "gene": "UniProtKB:Q9Y5B8",
  "gene_symbol": "NME7"
}